{
  "gene_name": "Protocadherin-8",
  "gene_symbol": "PCDH8",
  "gene": "UniProtKB:O95206",
  "term_id": "GO:0098609",
  "term_label": "cell-cell adhesion"
}